{
  "gene": "UniProtKB:P14859",
  "gene_symbol": "POU2F1",
  "gene_name": "POU domain, class 2, transcription factor 1",
  "term_id": "GO:0000978",
  "term_label": "RNA polymerase II cis-regulatory region sequence-specific DNA binding"
}